{
  "gene_name": "Putative KHDC1-like protein",
  "gene_symbol": "KHDC1L",
  "term_id": "UNKNOWN:0002",
  "gene": "UniProtKB:Q5JSQ8",
  "term_label": "Unknown biological process"
}